{
  "gene_name": "Oncostatin-M-specific receptor subunit beta",
  "gene": "UniProtKB:Q99650",
  "term_id": "GO:0004924",
  "term_label": "oncostatin-M receptor activity",
  "gene_symbol": "OSMR"
}